intracellular mRNA localization [GO:0008298] (biological process) Definition: Any process in which mRNA is transported to, or maintained in, a specific location within the cell. Relationships: is a type of GO:0006403 Also known as: establishment and maintenance of intracellular RNA localization, intracellular mRNA localisation, mRNA localization, intracellular, intracellular mRNA positioning, mRNA positioning, intracellular Subtypes: mRNA localization resulting in post-transcriptional regulation of gene expression [GO:0010609], GO:0060810 Regulation: regulated by regulation of intracellular mRNA localization [GO:1904580]; negatively regulated by negative regulation of intracellular mRNA localization [GO:1904581]; positively regulated by positive regulation of intracellular mRNA localization [GO:1904582] Sources: GOC:ai